{
  "term_id": "GO:0009897",
  "gene_name": "UL16-binding protein 6",
  "gene": "UniProtKB:Q5VY80",
  "term_label": "external side of plasma membrane",
  "gene_symbol": "RAET1L"
}